cellular response to interleukin-9 [GO:0071355] (biological process) Sources: GOC:mah Also known as: cellular response to IL-9 Relationships: is a type of GO:0071104; is a type of cellular response to cytokine stimulus [GO:0071345] Definition: Any process that results in a change in state or activity of a cell (in terms of movement, secretion, enzyme production, gene expression, etc.) as a result of an interleukin-9 stimulus.